{
  "gene_symbol": "ERRFI1",
  "gene": "UniProtKB:Q9UJM3",
  "term_id": "GO:0045616",
  "gene_name": "ERBB receptor feedback inhibitor 1",
  "term_label": "regulation of keratinocyte differentiation"
}